{
  "term_id": "GO:0043130",
  "gene_symbol": "UBXN8",
  "gene": "UniProtKB:O00124",
  "term_label": "ubiquitin binding",
  "gene_name": "UBX domain-containing protein 8"
}